{
  "gene_symbol": "NTRK2",
  "term_id": "GO:1990416",
  "gene_name": "BDNF_NT-3 growth factors receptor",
  "term_label": "cellular response to brain-derived neurotrophic factor stimulus",
  "gene": "UniProtKB:Q16620"
}